Isp3 layer of spore wall [GO:1990916] (cellular component) Relationships: is a type of cellular anatomical structure [GO:0110165]; is part of GO:0005619 Definition: The outermost layers of the spore wall, as described in Schizosaccharomyces pombe. References: PMID:24623719